renin-angiotensin regulation of aldosterone production [GO:0002018] (biological process) Definition: The process in which an increase in active angiotensin stimulates the adrenal cortices to secrete aldosterone. Sources: ISBN:0721643949 Also known as: renin-angiotensin control of aldosterone production Relationships: is a type of renal system process involved in regulation of systemic arterial blood pressure [GO:0003071]; is a type of GO:2000858; is part of GO:0002016